{
  "term_id": "GO:0005829",
  "gene": "UniProtKB:Q14195",
  "gene_name": "Dihydropyrimidinase-related protein 3",
  "term_label": "cytosol",
  "gene_symbol": "DPYSL3"
}